regulation of adenylate cyclase-inhibiting dopamine receptor signaling pathway [GO:1904990] (biological process) Definition: Any process that modulates the frequency, rate or extent of adenylate cyclase-inhibiting dopamine receptor signaling pathway. Subtypes: negative regulation of adenylate cyclase-inhibiting dopamine receptor signaling pathway [GO:1904991], positive regulation of adenylate cyclase-inhibiting dopamine receptor signaling pathway [GO:1904992] Relationships: is a type of regulation of dopamine receptor signaling pathway [GO:0060159]; regulates adenylate cyclase-inhibiting dopamine receptor signaling pathway [GO:0007195] Also known as: regulation of dopamine receptor, adenylate cyclase inhibiting pathway, regulation of dopamine receptor, adenylyl cyclase inhibiting pathway, regulation of inhibition of adenylate cyclase activity by dopamine receptor signalling pathway, regulation of inhibition of adenylate cyclase activity by dopamine receptor signaling pathway References: PMID:26554819 Sources: GOC:TermGenie, GOC:kmv, GO_REF:0000058